{
  "term_id": "GO:0000978",
  "gene": "UniProtKB:P08047",
  "gene_name": "Transcription factor Sp1",
  "term_label": "RNA polymerase II cis-regulatory region sequence-specific DNA binding",
  "gene_symbol": "SP1"
}